{
  "term_label": "Unknown cellular component",
  "gene_symbol": "LINC02902",
  "gene_name": "Putative uncharacterized protein LINC02902",
  "term_id": "UNKNOWN:0003",
  "gene": "UniProtKB:Q6ZTY9"
}